{
  "gene": "UniProtKB:O75586",
  "term_id": "GO:0070847",
  "term_label": "core mediator complex",
  "gene_symbol": "MED6",
  "gene_name": "Mediator of RNA polymerase II transcription subunit 6"
}